{
  "gene": "UniProtKB:P47992",
  "term_id": "GO:0008009",
  "term_label": "chemokine activity",
  "gene_symbol": "XCL1",
  "gene_name": "Lymphotactin"
}